{
  "term_id": "GO:0042147",
  "gene_symbol": "RAB9B",
  "gene_name": "Ras-related protein Rab-9B",
  "term_label": "retrograde transport, endosome to Golgi",
  "gene": "UniProtKB:Q9NP90"
}